dGDP biosynthetic process [GO:0006185] (biological process) Also known as: dGDP anabolism, dGDP biosynthesis, dGDP formation, dGDP synthesis Sources: ISBN:0198506732 Definition: The chemical reactions and pathways resulting in the formation of dGDP, deoxyguanosine diphosphate, (2'-deoxyguanosine 5'-diphosphate). Relationships: is a type of purine deoxyribonucleotide biosynthetic process [GO:0009153]; is a type of purine deoxyribonucleoside diphosphate biosynthetic process [GO:0009183]; is a type of GO:0046066